{
  "gene": "UniProtKB:P10451",
  "gene_symbol": "SPP1",
  "term_label": "extracellular space",
  "term_id": "GO:0005615",
  "gene_name": "Osteopontin"
}